{
  "gene_symbol": "ZDHHC2",
  "term_id": "GO:0005794",
  "gene_name": "Palmitoyltransferase ZDHHC2",
  "gene": "UniProtKB:Q9UIJ5",
  "term_label": "Golgi apparatus"
}